{
  "gene": "UniProtKB:P33552",
  "term_id": "GO:0019005",
  "gene_symbol": "CKS2",
  "gene_name": "Cyclin-dependent kinases regulatory subunit 2",
  "term_label": "SCF ubiquitin ligase complex"
}